{
  "gene_name": "ATP-dependent RNA helicase DHX33",
  "gene_symbol": "DHX33",
  "gene": "UniProtKB:Q9H6R0",
  "term_label": "helicase activity",
  "term_id": "GO:0004386"
}